C21-steroid hormone catabolic process [GO:0008208] (biological process) Definition: The chemical reactions and pathways resulting in the breakdown of C21-steroid hormones, steroid compounds containing 21 carbons which function as hormones. Sources: GOC:ai Also known as: C21-steroid hormone breakdown, C21-steroid hormone catabolism, C21-steroid hormone degradation Relationships: is a type of steroid catabolic process [GO:0006706]; is a type of C21-steroid hormone metabolic process [GO:0008207]; is a type of hormone catabolic process [GO:0042447] Subtypes: GO:0006709, aldosterone catabolic process [GO:0032343]